embryonic root morphogenesis [GO:0010086] (biological process) Definition: The process in which the anatomical structures of the embryonic root are generated and organized. Sources: GOC:tb Relationships: is a type of GO:0010015; is a type of embryonic morphogenesis [GO:0048598]